{
  "gene": "UniProtKB:Q96DU7",
  "gene_symbol": "ITPKC",
  "term_label": "inositol phosphate biosynthetic process",
  "term_id": "GO:0032958",
  "gene_name": "Inositol-trisphosphate 3-kinase C"
}